negative regulation of lens epithelial cell proliferation [GO:2001110] (biological process) Definition: Any process that stops, prevents or reduces the frequency, rate or extent of lens epithelial cell proliferation. Sources: GOC:obol Relationships: is a type of negative regulation of epithelial cell proliferation [GO:0050680]; is a type of negative regulation of multicellular organismal process [GO:0051241]; is a type of regulation of lens epithelial cell proliferation [GO:2001109]; negatively regulates GO:0097166